CCL2-activated CCR4 signaling pathway [GO:0038153] (biological process) Relationships: is a type of chemokine (C-C motif) ligand 2 signaling pathway [GO:0038148]; is a type of C-C chemokine receptor CCR4 signaling pathway [GO:0038152] Also known as: CCL2/CCR4 signaling pathway Sources: GOC:nhn, GOC:signaling Definition: The series of molecular signals initiated by the binding of the C-C chemokine CCL2 to a C-C chemokine type 4 receptor (CCR4) on the surface of a target cell, and ending with the regulation of a downstream cellular process, e.g. transcription.